{
  "gene_symbol": "MBD6",
  "gene_name": "Methyl-CpG-binding domain protein 6",
  "term_id": "UNKNOWN:0002",
  "gene": "UniProtKB:Q96DN6",
  "term_label": "Unknown biological process"
}